{
  "term_id": "GO:0008656",
  "gene_symbol": "CTSH",
  "gene": "UniProtKB:P09668",
  "term_label": "cysteine-type endopeptidase activator activity involved in apoptotic process",
  "gene_name": "Pro-cathepsin H"
}